{
  "gene_symbol": "PRKCSH",
  "gene": "UniProtKB:P14314",
  "term_label": "glucosidase II complex",
  "term_id": "GO:0017177",
  "gene_name": "Glucosidase 2 subunit beta"
}